monocarboxylate:sodium symporter activity [GO:0140161] (MF) Subtypes: gamma-aminobutyric acid:sodium:chloride symporter activity [GO:0005332], bile acid:sodium symporter activity [GO:0008508] References: PMID:15322102 Sources: GOC:ln Relationships: is a type of organic acid:sodium symporter activity [GO:0005343]; is a type of secondary active monocarboxylate transmembrane transporter activity [GO:0015355] Definition: Enables the transfer of a solute or solutes from one side of a membrane to the other according to the reaction: monocarboxylate(out) + Na+(out) = monocarboxylate(in) + Na+(in).